{
  "term_label": "GTP binding",
  "term_id": "GO:0005525",
  "gene": "UniProtKB:Q3ZCM7",
  "gene_name": "Tubulin beta-8 chain",
  "gene_symbol": "TUBB8"
}